{
  "term_label": "mitochondrion",
  "term_id": "GO:0005739",
  "gene": "UniProtKB:Q16773",
  "gene_name": "Kynurenine--oxoglutarate transaminase 1",
  "gene_symbol": "KYAT1"
}